{
  "gene_name": "Alpha-(1,3)-fucosyltransferase 10",
  "term_id": "UNKNOWN:0002",
  "term_label": "Unknown biological process",
  "gene_symbol": "FUT10",
  "gene": "UniProtKB:Q6P4F1"
}